{
  "gene_name": "SURP and G-patch domain-containing protein 2",
  "term_id": "GO:0003723",
  "gene_symbol": "SUGP2",
  "gene": "UniProtKB:Q8IX01",
  "term_label": "RNA binding"
}